{
  "gene_name": "Protein dopey-2",
  "gene_symbol": "DOP1B",
  "gene": "UniProtKB:Q9Y3R5",
  "term_label": "Unknown biological process",
  "term_id": "UNKNOWN:0002"
}